{
  "term_id": "GO:0019838",
  "gene": "UniProtKB:Q9BYJ0",
  "term_label": "growth factor binding",
  "gene_symbol": "FGFBP2",
  "gene_name": "Fibroblast growth factor-binding protein 2"
}